{
  "gene": "UniProtKB:Q86VY4",
  "term_label": "Unknown biological process",
  "gene_symbol": "TSPYL5",
  "term_id": "UNKNOWN:0002",
  "gene_name": "Testis-specific Y-encoded-like protein 5"
}